{
  "gene_symbol": "MAPKAPK2",
  "term_id": "GO:0005516",
  "gene_name": "MAP kinase-activated protein kinase 2",
  "gene": "UniProtKB:P49137",
  "term_label": "calmodulin binding"
}